{
  "gene_name": "Guanine nucleotide-binding protein G(i) subunit alpha-1",
  "term_id": "GO:0005834",
  "gene": "UniProtKB:P63096",
  "gene_symbol": "GNAI1",
  "term_label": "heterotrimeric G-protein complex"
}